regulation of heart induction [GO:0090381] (BP) Definition: Any process that modulates the rate, frequency, or extent of heart induction. Heart induction is the close range interaction between mesoderm and endoderm or ectoderm that causes cells to change their fates and specify the development of the heart. Relationships: is_a regulation of animal organ formation [GO:0003156]; is a type of regulation of multicellular organismal process [GO:0051239]; is a type of regulation of heart morphogenesis [GO:2000826]; regulates heart induction [GO:0003129] Sources: GOC:dph, GOC:tb Subtypes: GO:1901320, positive regulation of heart induction [GO:1901321]